{
  "gene_name": "Serine_threonine-protein kinase_endoribonuclease IRE1",
  "term_id": "GO:0004674",
  "gene": "UniProtKB:O75460",
  "term_label": "protein serine/threonine kinase activity",
  "gene_symbol": "ERN1"
}